{
  "gene": "UniProtKB:P10746",
  "gene_symbol": "Mgu",
  "gene_name": "Uroporphyrinogen-III synthase",
  "term_id": "GO:0004852",
  "term_label": "uroporphyrinogen-III synthase activity"
}